{
  "term_id": "GO:0005886",
  "gene_symbol": "CD63",
  "gene_name": "CD63 antigen",
  "gene": "UniProtKB:P08962",
  "term_label": "plasma membrane"
}